{
  "gene": "UniProtKB:O95363",
  "gene_name": "Phenylalanine--tRNA ligase, mitochondrial",
  "gene_symbol": "FARS2",
  "term_label": "cytoplasm",
  "term_id": "GO:0005737"
}